metanephric mesenchymal cell proliferation involved in metanephros development [GO:0072136] (biological process) Relationships: is a type of GO:0072135; is a type of GO:0072203; is part of metanephric mesenchyme development [GO:0072075] Definition: The multiplication or reproduction of cells, resulting in the expansion of a metanephric mesenchymal cell population. Sources: GOC:mtg_kidney_jan10